{
  "gene": "UniProtKB:O60229",
  "gene_symbol": "KALRN",
  "term_label": "cytoplasm",
  "term_id": "GO:0005737",
  "gene_name": "Kalirin"
}